{
  "gene_name": "Probable cytosolic iron-sulfur protein assembly protein CIAO1",
  "term_label": "cytosolic [4Fe-4S] assembly targeting complex",
  "term_id": "GO:0097361",
  "gene": "UniProtKB:O76071",
  "gene_symbol": "CIAO1"
}